glycine dehydrogenase (decarboxylating) activity [GO:0004375] (molecular function) Sources: RHEA:24304 Relationships: is a type of oxidoreductase activity, acting on the CH-NH2 group of donors, disulfide as acceptor [GO:0016642] Definition: Catalysis of the reaction: N(6)-[(R)-lipoyl]-L-lysyl-[glycine-cleavage complex H protein] + glycine + H+ = N(6)-[(R)-S(8)-aminomethyldihydrolipoyl]-L-lysyl-[glycine-cleavage complex H protein] + CO2. Also known as: P-protein, glycine cleavage system P-protein activity, protein P1, glycine decarboxylase activity, glycine-cleavage complex, glycine-cleavage complex P-protein activity, glycine:H-protein-lipoyllysine oxidoreductase (decarboxylating, acceptor-amino-methylating), glycine:lipoylprotein oxidoreductase (decarboxylating and acceptor-aminomethylating)